detection of gibberellic acid stimulus [GO:0009728] (biological process) Relationships: is_a detection of hormone stimulus [GO:0009720]; is a type of response to gibberellin [GO:0009739] Definition: The series of events in which a gibberellic acid stimulus is received by a cell and converted into a molecular signal. Also known as: perception of gibberellic acid stimulus Sources: GOC:sm